{
  "term_label": "angiotensin maturation",
  "term_id": "GO:0002003",
  "gene_name": "Glutamyl aminopeptidase",
  "gene": "UniProtKB:Q07075",
  "gene_symbol": "ENPEP"
}